{
  "gene": "UniProtKB:P53672",
  "term_label": "visual perception",
  "gene_symbol": "CRYBA2",
  "gene_name": "Beta-crystallin A2",
  "term_id": "GO:0007601"
}